{
  "gene_symbol": "TEX101",
  "term_label": "regulation of flagellated sperm motility",
  "gene_name": "Testis-expressed protein 101",
  "term_id": "GO:1901317",
  "gene": "UniProtKB:Q9BY14"
}